{
  "term_label": "negative regulation of transcription by RNA polymerase II",
  "gene": "UniProtKB:Q9HC78",
  "gene_symbol": "ZBTB20",
  "term_id": "GO:0000122",
  "gene_name": "Zinc finger and BTB domain-containing protein 20"
}